{
  "gene_name": "Negative elongation factor B",
  "gene_symbol": "NELFB",
  "term_label": "Unknown molecular function",
  "term_id": "UNKNOWN:0001",
  "gene": "UniProtKB:Q8WX92"
}